positive regulation of organ growth [GO:0046622] (biological process) Subtypes: positive regulation of heart growth [GO:0060421] Definition: Any process that activates or increases the frequency, rate or extent of growth of an organ of an organism. Relationships: is a type of regulation of organ growth [GO:0046620]; is a type of positive regulation of developmental growth [GO:0048639]; is a type of positive regulation of multicellular organismal process [GO:0051240]; positively regulates organ growth [GO:0035265] Sources: GOC:bf, GOC:tb